cellular response to vitamin B1 starvation [GO:0036225] (biological process) Definition: Any process that results in a change in state or activity of a cell (in terms of movement, secretion, enzyme production, gene expression, etc.) as a result of deprivation of vitamin B1 (also called thiamin and thiamine). Sources: GOC:al, Wikipedia:Thiamine Also known as: cellular response to thiamin starvation, cellular response to vitamin B1 deprivation Relationships: is a type of cellular response to starvation [GO:0009267]